{
  "gene_name": "Endogenous retrovirus group K member 19 Pol protein",
  "gene": "UniProtKB:Q9WJR5",
  "term_id": "UNKNOWN:0002",
  "gene_symbol": "ERVK-19",
  "term_label": "Unknown biological process"
}